{
  "gene_symbol": "UBXN2A",
  "term_id": "GO:0061025",
  "term_label": "membrane fusion",
  "gene_name": "UBX domain-containing protein 2A",
  "gene": "UniProtKB:P68543"
}